L-glutamate import into mitochondrion [GO:0110141] (biological process) References: PMID:30297026 Sources: GOC:vw Relationships: is a type of L-glutamate transmembrane transport [GO:0015813] Definition: The process in which L-glutamate is transported from the cytosol into the mitochondrial matrix.